regulation of nematode pharyngeal pumping [GO:0043051] (biological process) Subtypes: negative regulation of nematode pharyngeal pumping [GO:1903745], positive regulation of nematode pharyngeal pumping [GO:1903746] Relationships: is a type of GO:1903998; regulates nematode pharyngeal pumping [GO:0043050] References: PMID:2181052 Sources: GOC:cab1 Definition: Any process that modulates the contraction and relaxation movements of the pharyngeal muscle that mediates feeding in nematodes.